{
  "term_id": "GO:0032880",
  "gene_name": "Afadin",
  "gene_symbol": "AFDN",
  "gene": "UniProtKB:P55196",
  "term_label": "regulation of protein localization"
}